{
  "gene": "UniProtKB:Q99626",
  "term_id": "GO:0005634",
  "term_label": "nucleus",
  "gene_name": "Homeobox protein CDX-2",
  "gene_symbol": "CDX2"
}